pyrimidine nucleotide binding [GO:0019103] (molecular function) Sources: GOC:ai Relationships: is a type of nucleotide binding [GO:0000166] Subtypes: GO:0032556, pyrimidine ribonucleotide binding [GO:0032557] Definition: Binding to a pyrimidine nucleotide, a pyrimidine nucleoside esterified with (ortho)phosphate.